{
  "gene_symbol": "METTL27",
  "gene": "UniProtKB:Q8N6F8",
  "term_label": "Unknown biological process",
  "term_id": "UNKNOWN:0002",
  "gene_name": "Methyltransferase-like protein 27"
}